{
  "gene_name": "Protocadherin gamma-B2",
  "gene_symbol": "PCDHGB2",
  "gene": "UniProtKB:Q9Y5G2",
  "term_label": "cell adhesion molecule binding",
  "term_id": "GO:0050839"
}